{
  "gene_symbol": "MLIP",
  "term_id": "UNKNOWN:0001",
  "gene": "UniProtKB:Q5VWP3",
  "term_label": "Unknown molecular function",
  "gene_name": "Muscular LMNA-interacting protein"
}